{
  "gene_name": "Mitogen-activated protein kinase 6",
  "term_label": "cytoplasm",
  "term_id": "GO:0005737",
  "gene": "UniProtKB:Q16659",
  "gene_symbol": "MAPK6"
}